{
  "gene": "UniProtKB:P25713",
  "gene_name": "Metallothionein-3",
  "gene_symbol": "MT3",
  "term_id": "GO:0046872",
  "term_label": "metal ion binding"
}